{
  "gene_symbol": "FOXN3",
  "term_label": "DNA-binding transcription factor activity",
  "gene_name": "Forkhead box protein N3",
  "term_id": "GO:0003700",
  "gene": "UniProtKB:O00409"
}